pyrimidine nucleotide-sugar transmembrane transporter activity [GO:0015165] (molecular function) Relationships: is_a nucleotide-sugar transmembrane transporter activity [GO:0005338]; is part of GO:0090481 Sources: GOC:ai, GOC:mtg_transport, ISBN:0815340729 Definition: Enables the transfer of a pyrimidine nucleotide-sugar from one side of a membrane to the other. Pyrimidine nucleotide-sugars are pyrimidine nucleotides in glycosidic linkage with a monosaccharide or monosaccharide derivative. Subtypes: CMP-N-acetylneuraminate transmembrane transporter activity [GO:0005456], UDP-galactose transmembrane transporter activity [GO:0005459], UDP-glucose transmembrane transporter activity [GO:0005460], UDP-glucuronate transmembrane transporter activity [GO:0005461], UDP-N-acetylglucosamine transmembrane transporter activity [GO:0005462], UDP-N-acetylgalactosamine transmembrane transporter activity [GO:0005463], GO:0005464, UDP-beta-L-arabinofuranose transporter activity [GO:0140819]